{
  "gene_name": "Zinc finger protein basonuclin-2",
  "gene": "UniProtKB:Q6ZN30",
  "gene_symbol": "BNC2",
  "term_id": "GO:0006355",
  "term_label": "regulation of DNA-templated transcription"
}